{
  "gene_symbol": "CD6",
  "term_label": "lipopolysaccharide-mediated signaling pathway",
  "gene_name": "T-cell differentiation antigen CD6",
  "term_id": "GO:0031663",
  "gene": "UniProtKB:P30203"
}